{
  "gene": "UniProtKB:O95238",
  "gene_symbol": "SPDEF",
  "term_label": "DNA-binding transcription factor activity, RNA polymerase II-specific",
  "gene_name": "SAM pointed domain-containing Ets transcription factor",
  "term_id": "GO:0000981"
}